{
  "term_label": "Unknown cellular component",
  "gene": "UniProtKB:O43680",
  "gene_name": "Transcription factor 21",
  "term_id": "UNKNOWN:0003",
  "gene_symbol": "TCF21"
}